regulation of retrograde dense core granule transport [GO:1901954] (biological process) References: PMID:23358451 Sources: GOC:TermGenie, GOC:kmv Definition: Any process that modulates the frequency, rate or extent of retrograde dense core granule transport. Relationships: is a type of GO:1901608; is a type of GO:1904809; is a type of regulation of retrograde axon cargo transport [GO:2001017]; regulates retrograde neuronal dense core vesicle transport [GO:1990049] Subtypes: GO:1901955, positive regulation of retrograde dense core granule transport [GO:1901956]